cellular response to caloric restriction [GO:0061433] (biological process) Relationships: is a type of GO:0033554; is a type of response to caloric restriction [GO:0061771] Definition: Any process that results in a change in state or activity of a cell or an organism (in terms of movement, secretion, enzyme production, gene expression, etc.) as a result of a of caloric restriction, insufficient food energy intake. References: PMID:17914901 Sources: GOC:dph